{
  "gene": "UniProtKB:P48382",
  "term_label": "DNA-binding transcription factor activity, RNA polymerase II-specific",
  "gene_name": "DNA-binding protein RFX5",
  "gene_symbol": "RFX5",
  "term_id": "GO:0000981"
}